glucose-6-phosphate dehydrogenase (coenzyme F420) activity [GO:0052749] (molecular function) Relationships: is a type of oxidoreductase activity, acting on CH-OH group of donors [GO:0016614] Also known as: D-glucose-6-phosphate:F420 1-oxidoreductase activity, F420-dependent glucose-6-phosphate dehydrogenase activity, coenzyme F420-dependent glucose-6-phosphate dehydrogenase activity Definition: Catalysis of the reaction: beta-D-glucose 6-phosphate + coenzyme F420 + H+ = 6-O-phosphono-D-glucono-1,5-lactone + reduced coenzyme F420. Sources: EC:1.1.98.2, GOC:mengo_curators, RHEA:27294